{
  "gene_name": "Stathmin",
  "term_label": "microtubule depolymerization",
  "term_id": "GO:0007019",
  "gene": "UniProtKB:P16949",
  "gene_symbol": "STMN1"
}